{
  "term_id": "GO:0031012",
  "gene_name": "A disintegrin and metalloproteinase with thrombospondin motifs 12",
  "gene": "UniProtKB:P58397",
  "gene_symbol": "ADAMTS12",
  "term_label": "extracellular matrix"
}